regulation of lipoprotein oxidation [GO:0034442] (biological process) Relationships: is a type of regulation of lipoprotein metabolic process [GO:0050746]; regulates lipoprotein oxidation [GO:0042161] Sources: GOC:BHF, GOC:mah Subtypes: negative regulation of lipoprotein oxidation [GO:0034443], regulation of lipoprotein lipid oxidation [GO:0060587] Definition: Any process that modulates the frequency, rate or extent of lipoprotein oxidation.